{
  "gene_name": "Nanos homolog 2",
  "gene": "UniProtKB:P60321",
  "term_label": "mRNA binding",
  "term_id": "GO:0003729",
  "gene_symbol": "NANOS2"
}